{
  "gene_symbol": "CRP",
  "gene_name": "C-reactive protein",
  "term_id": "GO:0005615",
  "gene": "UniProtKB:P02741",
  "term_label": "extracellular space"
}